microtubule [GO:0005874] (cellular component) Definition: Any of the long, generally straight, hollow tubes of internal diameter 12-15 nm and external diameter 24 nm found in a wide variety of eukaryotic cells; each consists (usually) of 13 protofilaments of polymeric tubulin, staggered in such a manner that the tubulin monomers are arranged in a helical pattern on the microtubular surface, and with the alpha/beta axes of the tubulin subunits parallel to the long axis of the tubule; exist in equilibrium with pool of tubulin monomers and can be rapidly assembled or disassembled in response to physiological stimuli; concerned with force generation, e.g. in the spindle. Sources: ISBN:0879693568 Subtypes: spindle microtubule [GO:0005876], nuclear microtubule [GO:0005880], GO:0005881, subpellicular microtubule [GO:0020025], intraconoid microtubule [GO:0033289], dendritic microtubule [GO:1901588], post-anaphase array microtubule [GO:1905759] Also known as: microtubuli, microtubulus, neurotubule Relationships: is_a polymeric cytoskeletal fiber [GO:0099513]; is part of microtubule cytoskeleton [GO:0015630]